protein sialylation [GO:1990743] (biological process) Definition: A protein modification process that results in the addition of a sialic acid unit to the end of an oligosaccharide chain in a glycoprotein. References: PMID:21930713 Relationships: is a type of protein modification process [GO:0036211]; is a type of sialylation [GO:0097503]